oxidoreductase activity, acting on NAD(P)H, oxygen as acceptor [GO:0050664] (molecular function) Definition: Catalysis of an oxidation-reduction (redox) reaction in which NADH or NADPH acts as a hydrogen or electron donor and reduces an oxygen molecule. Relationships: is a type of oxidoreductase activity, acting on NAD(P)H [GO:0016651] Also known as: oxidoreductase activity, acting on NADH or NADPH, oxygen as acceptor Subtypes: GO:0016174, GO:0016175 Sources: EC:1.6.3.-